ent-cassa-12,15-diene 11-hydroxylase activity [GO:0036202] (molecular function) Relationships: is a type of oxidoreductase activity, acting on paired donors, with incorporation or reduction of molecular oxygen, NAD(P)H as one donor, and incorporation of one atom of oxygen [GO:0016709] Also known as: ent-cassadiene C11alpha-hydroxylase activity Definition: Catalysis of the reaction: ent-cassa-12,15-diene + O2 + NADPH + H+ = ent-11beta-hydroxycassa-12,15-diene + NADP+ + H2O. Sources: EC:1.14.14.112